{
  "term_label": "RNA polymerase II cis-regulatory region sequence-specific DNA binding",
  "gene_symbol": "ZNF691",
  "gene": "UniProtKB:Q5VV52",
  "gene_name": "Zinc finger protein 691",
  "term_id": "GO:0000978"
}